{
  "gene": "UniProtKB:Q6IQ26",
  "gene_name": "DENN domain-containing protein 5A",
  "gene_symbol": "DENND5A",
  "term_label": "trans-Golgi network",
  "term_id": "GO:0005802"
}